{
  "gene": "UniProtKB:Q6ISB3",
  "gene_name": "Grainyhead-like protein 2 homolog",
  "gene_symbol": "GRHL2",
  "term_id": "GO:0006357",
  "term_label": "regulation of transcription by RNA polymerase II"
}